{
  "term_id": "GO:0005634",
  "gene_name": "CREB-regulated transcription coactivator 3",
  "gene": "UniProtKB:Q6UUV7",
  "gene_symbol": "CRTC3",
  "term_label": "nucleus"
}